response to arsenite ion [GO:1903842] (biological process) Definition: Any process that results in a change in state or activity of a cell or an organism (in terms of movement, secretion, enzyme production, gene expression, etc.) as a result of an arsenite ion stimulus. Subtypes: cellular response to arsenite ion [GO:1903843] Relationships: is a type of response to arsenic-containing substance [GO:0046685]; is a type of response to oxygen-containing compound [GO:1901700] References: PMID:12106899 Sources: GOC:TermGenie, GOC:mr, GO_REF:0000071